{
  "term_id": "GO:0004984",
  "gene_name": "Olfactory receptor",
  "gene_symbol": "LOC112268384",
  "term_label": "olfactory receptor activity",
  "gene": "UniProtKB:A0A2R8YEH3"
}